{
  "gene_name": "Cholesteryl ester transfer protein",
  "term_label": "triglyceride metabolic process",
  "gene": "UniProtKB:P11597",
  "term_id": "GO:0006641",
  "gene_symbol": "CETP"
}